ethylene biosynthesis involved in jasmonic acid and ethylene-dependent systemic resistance [GO:0043272] (biological process) Definition: The chemical reactions and pathways resulting in the formation of ethylene (C2-H4, ethene), occurring as part of the process of jasmonic acid and ethylene-dependent systemic resistance. Sources: GOC:jl Relationships: is a type of ethylene biosynthetic process [GO:0009693]; is part of jasmonic acid and ethylene-dependent systemic resistance [GO:0009861] Also known as: ethylene anabolism during jasmonic acid and ethylene-dependent systemic resistance, ethylene biosynthetic process during jasmonic acid and ethylene-dependent systemic resistance, ethylene formation during jasmonic acid and ethylene-dependent systemic resistance, ethylene synthesis during jasmonic acid and ethylene-dependent systemic resistance